muscle cell chemotaxis toward tendon cell [GO:0036061] (biological process) Also known as: muscle cell chemotaxis towards tendon cell, muscle cell attraction References: PMID:19793885 Sources: GOC:sart Relationships: is a type of muscle cell migration [GO:0014812]; is a type of GO:0060326 Definition: The directed movement of a muscle cell towards a tendon cell in response to an external stimulus. Tendon cells, for example, produce positive guidance cues that attract muscle cells. Regulation: regulated by regulation of muscle cell chemotaxis toward tendon cell [GO:2001281]; negatively regulated by negative regulation of muscle cell chemotaxis toward tendon cell [GO:2001282]